regulation of fibroblast growth factor receptor signaling pathway involved in ureteric bud formation [GO:2000702] (biological process) Definition: Any process that modulates the frequency, rate or extent of fibroblast growth factor receptor signaling pathway involved in ureteric bud formation. Sources: GOC:mtg_kidney_jan10, GOC:obol, GOC:yaf Also known as: regulation of FGF receptor signaling pathway of ureteric bud formation, regulation of FGF receptor signalling pathway of ureteric bud formation, regulation of FGFR signaling pathway of ureteric bud formation, regulation of fibroblast growth factor receptor signaling pathway of ureteric bud formation, regulation of fibroblast growth factor receptor signalling pathway of ureteric bud formation Relationships: is a type of regulation of fibroblast growth factor receptor signaling pathway [GO:0040036]; regulates fibroblast growth factor receptor signaling pathway involved in ureteric bud formation [GO:2000699] Subtypes: negative regulation of fibroblast growth factor receptor signaling pathway involved in ureteric bud formation [GO:2000703], positive regulation of fibroblast growth factor receptor signaling pathway involved in ureteric bud formation [GO:2000704]